{
  "gene_symbol": "PLEKHA3",
  "gene": "UniProtKB:Q9HB20",
  "gene_name": "Pleckstrin homology domain-containing family A member 3",
  "term_id": "GO:0005802",
  "term_label": "trans-Golgi network"
}